{
  "term_id": "GO:0060337",
  "gene_name": "Interferon alpha-2",
  "gene": "UniProtKB:P01563",
  "term_label": "type I interferon-mediated signaling pathway",
  "gene_symbol": "IFNA2"
}